{
  "gene_symbol": "CETP",
  "term_id": "GO:0034372",
  "term_label": "very-low-density lipoprotein particle remodeling",
  "gene": "UniProtKB:P11597",
  "gene_name": "Cholesteryl ester transfer protein"
}